negative regulation of gamma-delta T cell activation involved in immune response [GO:2001192] (biological process) Sources: GOC:obol Definition: Any process that stops, prevents or reduces the frequency, rate or extent of gamma-delta T cell activation involved in immune response. Relationships: is a type of negative regulation of immune effector process [GO:0002698]; is a type of GO:0046644; is a type of negative regulation of immune response [GO:0050777]; is a type of regulation of gamma-delta T cell activation involved in immune response [GO:2001191]; RO_0002212 gamma-delta T cell activation involved in immune response [GO:0002290] Also known as: negative regulation of gamma-delta T cell activation during immune response, negative regulation of gamma-delta T lymphocyte activation during immune response, negative regulation of gamma-delta T-cell activation during immune response, negative regulation of gamma-delta T-lymphocyte activation during immune response